{
  "gene": "UniProtKB:Q01196",
  "gene_symbol": "RUNX1",
  "term_label": "DNA-binding transcription factor activity, RNA polymerase II-specific",
  "term_id": "GO:0000981",
  "gene_name": "Runt-related transcription factor 1"
}